iron ion sequestering activity [GO:0140315] (molecular function) References: PMID:27780864 Definition: Binding to an iron ion to prevent it from interacting with other partners or to inhibit its localization to the area of the cell or complex where it is active. Relationships: is a type of metal ion sequestering activity [GO:0140487]; has part GO:0005506